{
  "gene_symbol": "SH3GLB1",
  "term_label": "protein-macromolecule adaptor activity",
  "gene_name": "Endophilin-B1",
  "gene": "UniProtKB:Q9Y371",
  "term_id": "GO:0030674"
}